{
  "term_label": "nucleus",
  "term_id": "GO:0005634",
  "gene": "UniProtKB:Q13490",
  "gene_name": "Baculoviral IAP repeat-containing protein 2",
  "gene_symbol": "BIRC2"
}